{
  "term_label": "Unknown molecular function",
  "gene": "UniProtKB:Q96CB8",
  "term_id": "UNKNOWN:0001",
  "gene_symbol": "INTS12",
  "gene_name": "Integrator complex subunit 12"
}